{
  "term_label": "UDP-N-acetylglucosamine metabolic process",
  "gene_symbol": "GFPT2",
  "gene": "UniProtKB:O94808",
  "term_id": "GO:0006047",
  "gene_name": "Glutamine--fructose-6-phosphate aminotransferase [isomerizing] 2"
}